{
  "term_label": "positive regulation of Arp2/3 complex-mediated actin nucleation",
  "gene": "UniProtKB:Q92558",
  "term_id": "GO:2000601",
  "gene_symbol": "WASF1",
  "gene_name": "Actin-binding protein WASF1"
}